{
  "term_label": "Unknown biological process",
  "gene": "UniProtKB:Q8TD35",
  "gene_name": "Protein LKAAEAR1",
  "term_id": "UNKNOWN:0002",
  "gene_symbol": "LKAAEAR1"
}